positive regulation of protein localization to ciliary membrane [GO:1903569] (biological process) Definition: Any process that activates or increases the frequency, rate or extent of protein localization to ciliary membrane. Also known as: positive regulation of protein localisation in ciliary membrane, positive regulation of protein localisation to ciliary membrane, positive regulation of protein localization in ciliary membrane, up regulation of protein localisation in ciliary membrane, up regulation of protein localisation to ciliary membrane, up regulation of protein localization in ciliary membrane, up regulation of protein localization to ciliary membrane, up-regulation of protein localisation in ciliary membrane, up-regulation of protein localisation to ciliary membrane, up-regulation of protein localization in ciliary membrane, up-regulation of protein localization to ciliary membrane, upregulation of protein localisation in ciliary membrane, upregulation of protein localisation to ciliary membrane, upregulation of protein localization in ciliary membrane, upregulation of protein localization to ciliary membrane, activation of protein localisation in ciliary membrane, activation of protein localisation to ciliary membrane, activation of protein localization in ciliary membrane, activation of protein localization to ciliary membrane References: PMID:22072986 Sources: GOC:TermGenie, GOC:cilia, GOC:krc, GO_REF:0000058 Relationships: is a type of positive regulation of protein localization to cilium [GO:1903566]; is a type of GO:1903567; is a type of GO:1904377; is a type of positive regulation of protein localization to membrane [GO:1905477]; positively regulates protein localization to ciliary membrane [GO:1903441]